{
  "term_id": "GO:0034722",
  "term_label": "gamma-glutamyl-peptidase activity",
  "gene_name": "Gamma-glutamyl hydrolase",
  "gene": "UniProtKB:Q92820",
  "gene_symbol": "GGH"
}